{
  "gene_name": "Endogenous retrovirus group V member 1 Env polyprotein",
  "term_id": "UNKNOWN:0003",
  "term_label": "Unknown cellular component",
  "gene": "UniProtKB:B6SEH8",
  "gene_symbol": "ERVV-1"
}